{
  "term_label": "GTP binding",
  "gene_symbol": "RHOU",
  "term_id": "GO:0005525",
  "gene": "UniProtKB:Q7L0Q8",
  "gene_name": "Rho-related GTP-binding protein RhoU"
}